male germ-line sex determination [GO:0019100] (biological process) Sources: GOC:mah Definition: The determination of sex and sexual phenotype in a male organism's germ line. Relationships: is a type of GO:0007542; is a type of GO:0018992; is a type of male sex determination [GO:0030238]